norepinephrine binding [GO:0051380] (molecular function) Relationships: is a type of GO:0043169; is a type of GO:1901338 Sources: GOC:ai Also known as: noradrenaline binding Definition: Binding to norepinephrine, (3,4-dihydroxyphenyl-2-aminoethanol), a hormone secreted by the adrenal medulla and a neurotransmitter in the sympathetic peripheral nervous system and in some tracts of the CNS. It is also the biosynthetic precursor of epinephrine.